{
  "term_label": "mitochondrial ribosome assembly",
  "gene": "UniProtKB:Q96I51",
  "term_id": "GO:0061668",
  "gene_symbol": "RCC1L",
  "gene_name": "RCC1-like G exchanging factor-like protein"
}